ionotropic olfactory receptor activity [GO:0170020] (molecular function) Definition: Enables the transmembrane transfer of an ion by a channel that opens when a specific odorant has been bound by the channel complex or one of its constituent parts. Relationships: is a type of olfactory receptor activity [GO:0004984]; is a type of GO:0015276 References: PMID:21857978, PMID:24661599